response to luteinizing hormone [GO:0034699] (biological process) Also known as: response to luteinizing hormone stimulus Relationships: is a type of response to gonadotropin [GO:0034698]; is_a response to peptide hormone [GO:0043434] Subtypes: cellular response to luteinizing hormone stimulus [GO:0071373] Definition: Any process that results in a change in state or activity of a cell or an organism (in terms of movement, secretion, enzyme production, gene expression, etc.) as a result of a luteinizing hormone stimulus. Sources: GOC:BHF, GOC:vk